{
  "term_label": "arylsulfatase activity",
  "gene": "UniProtKB:Q5FYA8",
  "term_id": "GO:0004065",
  "gene_name": "Arylsulfatase H",
  "gene_symbol": "ARSH"
}